{
  "term_id": "UNKNOWN:0001",
  "gene": "UniProtKB:Q8NBT3",
  "gene_symbol": "TMEM145",
  "gene_name": "Transmembrane protein 145",
  "term_label": "Unknown molecular function"
}